spindle [GO:0005819] (cellular component) Subtypes: mitotic spindle [GO:0072686], meiotic spindle [GO:0072687] Sources: ISBN:0198547684 Relationships: is a type of intracellular membraneless organelle [GO:0043232]; BFO_0000050 GO:0015630 Definition: The array of microtubules and associated molecules that forms between opposite poles of a eukaryotic cell during mitosis or meiosis and serves to move the duplicated chromosomes apart.